egg-laying behavior [GO:0018991] (biological process) Relationships: is_a reproductive behavior [GO:0019098] References: PMID:18050396, PMID:31164023 Sources: GOC:ems Definition: A reproductive behavior that results in the deposition of eggs (either fertilized or not) upon a surface or into a medium such as water. Also known as: egg laying, egg-laying, oviposition, post-mating oviposition Regulation: regulated by GO:0046662; negatively regulated by negative regulation of egg-laying behavior [GO:1901045]; positively regulated by positive regulation of egg-laying behavior [GO:1901046]